vacuole-mitochondrion membrane contact site [GO:1990816] (cellular component) Also known as: vCLAMP, vacuole and mitochondria patch References: PMID:25026035, PMID:25026036 Relationships: is a type of organelle membrane contact site [GO:0044232] Definition: A zone of apposition between the vacuolar membrane and the mitochondrial outer membrane, important for transfer of lipids between the two organelles.